troponin complex [GO:0005861] (cellular component) Relationships: is a type of protein-containing complex [GO:0032991]; is part of GO:0005865 Sources: ISBN:0815316194 Definition: A complex of accessory proteins (typically troponin T, troponin I and troponin C) found associated with actin in muscle thin filaments; involved in calcium regulation of muscle contraction. Subtypes: cardiac Troponin complex [GO:1990584]